{
  "term_id": "GO:0001992",
  "gene_symbol": "OXTR",
  "gene_name": "Oxytocin receptor",
  "gene": "UniProtKB:P30559",
  "term_label": "regulation of systemic arterial blood pressure by vasopressin"
}